mucocyst [GO:0036000] (CC) References: PMID:10723937, PMID:4629881 Sources: GOC:mag Relationships: is a type of secretory granule [GO:0030141] Definition: A small subcellular vesicle, surrounded by a membrane, in the pellicle of ciliate protozoans that discharges a mucus-like secretion.